negative regulation of zinc ion transmembrane transport [GO:0071583] (biological process) Definition: Any process that stops, prevents, or reduces the frequency, rate or extent of the directed movement of zinc ions (Zn2+) from one side of a membrane to the other. Sources: GOC:BHF, GOC:mah Also known as: negative regulation of zinc ion membrane transport Relationships: is a type of GO:0071580; is a type of negative regulation of zinc ion transport [GO:0071582]; is a type of negative regulation of cation transmembrane transport [GO:1904063]; negatively regulates zinc ion transmembrane transport [GO:0071577] Subtypes: GO:0071584